{
  "term_label": "cilium-dependent cell motility",
  "gene_name": "EF-hand domain-containing protein 1",
  "gene_symbol": "EFHC1",
  "gene": "UniProtKB:Q5JVL4",
  "term_id": "GO:0060285"
}